{
  "gene_symbol": "ZNF423",
  "term_label": "Unknown cellular component",
  "gene_name": "Zinc finger protein 423",
  "term_id": "UNKNOWN:0003",
  "gene": "UniProtKB:Q2M1K9"
}